positive regulation of UDP-N-acetylglucosamine biosynthetic process [GO:0106280] (biological process) Also known as: positive egulation of UDP-N-acetylglucosamine formation, positive regulation of UDP-GlcNAc biosynthetic process, positive regulation of UDP-N-acetylglucosamine anabolism, positive regulation of UDP-N-acetylglucosamine biosynthesis, positive regulation of UDP-N-acetylglucosamine synthesis Definition: Any process that activates or increases the frequency, rate or extent of the UDP-N-acetylglucosamine biosynthetic process. Relationships: is a type of positive regulation of biosynthetic process [GO:0009891]; is a type of positive regulation of phosphate metabolic process [GO:0045937]; is a type of positive regulation of small molecule metabolic process [GO:0062013]; is a type of regulation of UDP-N-acetylglucosamine biosynthetic process [GO:0106278]; positively regulates UDP-N-acetylglucosamine biosynthetic process [GO:0006048] References: PMID:32579556